{
  "term_label": "nuclear pore localization",
  "term_id": "GO:0051664",
  "gene": "UniProtKB:P20700",
  "gene_symbol": "LMNB1",
  "gene_name": "Lamin-B1"
}